{
  "term_label": "cell adhesion",
  "term_id": "GO:0007155",
  "gene_symbol": "SRC",
  "gene": "UniProtKB:P12931",
  "gene_name": "Proto-oncogene tyrosine-protein kinase Src"
}